{
  "term_label": "plasma membrane",
  "gene_symbol": "OR10J6P",
  "gene_name": "Putative olfactory receptor 10J6",
  "gene": "UniProtKB:Q8NGY7",
  "term_id": "GO:0005886"
}